sterol transport [GO:0015918] (BP) Sources: GOC:ai Definition: The directed movement of sterols into, out of or within a cell, or between cells, by means of some agent such as a transporter or pore. Sterols are steroids with one or more hydroxyl groups and a hydrocarbon side-chain in the molecule. Relationships: is_a lipid transport [GO:0006869]; is a type of organic hydroxy compound transport [GO:0015850] Subtypes: cholesterol transport [GO:0030301], intracellular sterol transport [GO:0032366], sterol import [GO:0035376], sterol transmembrane transport [GO:0035382], intermembrane sterol transfer [GO:0120011] Regulation: regulated by GO:0032371; negatively regulated by negative regulation of sterol transport [GO:0032372]; positively regulated by positive regulation of sterol transport [GO:0032373]